{
  "gene_symbol": "IER5L",
  "gene_name": "Immediate early response gene 5-like protein",
  "term_id": "UNKNOWN:0002",
  "gene": "UniProtKB:Q5T953",
  "term_label": "Unknown biological process"
}